{
  "gene": "UniProtKB:Q9NPD5",
  "gene_name": "Solute carrier organic anion transporter family member 1B3",
  "gene_symbol": "SLCO1B3",
  "term_label": "sodium-independent organic anion transport",
  "term_id": "GO:0043252"
}